{
  "term_id": "GO:0000176",
  "gene_symbol": "DIS3",
  "gene": "UniProtKB:Q9Y2L1",
  "gene_name": "Exosome complex exonuclease RRP44",
  "term_label": "nuclear exosome (RNase complex)"
}